cellular response to mannitol stimulus [GO:0071325] (biological process) Relationships: is a type of GO:0010555; is a type of cellular response to carbohydrate stimulus [GO:0071322] Sources: GOC:mah Definition: Any process that results in a change in state or activity of a cell (in terms of movement, secretion, enzyme production, gene expression, etc.) as a result of a mannitol stimulus.